{
  "term_label": "membrane raft",
  "gene_name": "Amyloid-beta precursor protein",
  "term_id": "GO:0045121",
  "gene_symbol": "APP",
  "gene": "UniProtKB:P05067"
}